{
  "gene_symbol": "CRTC1",
  "gene_name": "CREB-regulated transcription coactivator 1",
  "term_id": "GO:0008140",
  "gene": "UniProtKB:Q6UUV9",
  "term_label": "cAMP response element binding protein binding"
}